{
  "gene_symbol": "LSM1",
  "term_id": "GO:1990726",
  "gene_name": "U6 snRNA-associated Sm-like protein LSm1",
  "term_label": "Lsm1-7-Pat1 complex",
  "gene": "UniProtKB:O15116"
}